{
  "gene_symbol": "CST7",
  "gene": "UniProtKB:O76096",
  "gene_name": "Cystatin-F",
  "term_label": "Golgi apparatus",
  "term_id": "GO:0005794"
}